vestibular nucleus development [GO:0021750] (biological process) Relationships: is a type of neural nucleus development [GO:0048857]; BFO_0000050 pons development [GO:0021548]; is part of GO:0021550 References: PMID:16221589 Sources: GOC:cls, GOC:curators, GOC:dgh, GOC:dph, GOC:jid Definition: The process whose specific outcome is the progression of the vestibular nucleus over time, from its formation to the mature structure.